microtubule-dependent intracellular transport of viral material [GO:0075519] (BP) Relationships: is a type of intracellular transport of virus [GO:0075733] Definition: The directed movement of the viral genome or viral particle within the host cell cytoplasm along host microtubules. Microtubule-dependent transport involves motor proteins like dynein and kinesin and is mostly used by viruses that target their genomes to the nucleus. Subtypes: microtubule-dependent intracellular transport of viral material towards cell periphery [GO:0039701], microtubule-dependent intracellular transport of viral material towards nucleus [GO:0075521] Sources: VZ:983